{
  "term_label": "microtubule cytoskeleton",
  "gene_name": "Cytosolic carboxypeptidase 3",
  "gene_symbol": "AGBL3",
  "gene": "UniProtKB:Q8NEM8",
  "term_id": "GO:0015630"
}